symbiont entry into host [GO:0044409] (biological process) Definition: Entry of a symbiont into the body, tissues, or cells of a host organism as part of the symbiont life cycle. The host is defined as the larger of the organisms involved in a symbiotic interaction. Sources: GOC:vw Also known as: entry into host, host invasion, host penetration, invasion into host, invasion of host, penetration into host, entry into cell of other organism during symbiotic interaction, entry into host cell via penetration peg, entry into host via a specialized structure during symbiotic interaction, entry into host via enzymatic degradation of host anatomical structure, entry into host via enzymatic degradation of host cuticle, penetration into host via a specialized structure, penetration into host via a specialized structure during symbiotic interaction, entry into cell of other organism involved in symbiotic interaction, entry into host through host barriers, entry into other organism during symbiotic interaction, entry into other organism involved in symbiotic interaction, invasion into other organism, invasion of other organism, invasive growth, other organism invasion Relationships: is a type of GO:0051701 Subtypes: entry of bacterium into host cell [GO:0035635], symbiont entry into host cell [GO:0046718], GO:0120326, entry into host through the stromata [GO:0140717] Regulation: regulated by modulation by symbiont of entry into host [GO:0052372]; positively regulated by positive regulation by symbiont of entry into host [GO:0075294]